tRNA aminoacylation for mitochondrial protein translation [GO:0070127] (biological process) Relationships: is a type of GO:0000959; is a type of tRNA aminoacylation for protein translation [GO:0006418]; BFO_0000050 mitochondrial translation [GO:0032543] Sources: GOC:mah Subtypes: mitochondrial alanyl-tRNA aminoacylation [GO:0070143], mitochondrial arginyl-tRNA aminoacylation [GO:0070144], mitochondrial asparaginyl-tRNA aminoacylation [GO:0070145], mitochondrial aspartyl-tRNA aminoacylation [GO:0070146], GO:0070147, mitochondrial glutaminyl-tRNA aminoacylation [GO:0070148], mitochondrial glutamyl-tRNA aminoacylation [GO:0070149], mitochondrial glycyl-tRNA aminoacylation [GO:0070150], GO:0070151, mitochondrial isoleucyl-tRNA aminoacylation [GO:0070152], mitochondrial leucyl-tRNA aminoacylation [GO:0070153], mitochondrial lysyl-tRNA aminoacylation [GO:0070154], mitochondrial methionyl-tRNA aminoacylation [GO:0070155], GO:0070156, mitochondrial prolyl-tRNA aminoacylation [GO:0070157], GO:0070158, GO:0070159, mitochondrial tryptophanyl-tRNA aminoacylation [GO:0070183], mitochondrial tyrosyl-tRNA aminoacylation [GO:0070184], GO:0070185 Definition: The synthesis of aminoacyl tRNA by the formation of an ester bond between the 3'-hydroxyl group of the most 3' adenosine of the tRNA, to be used in ribosome-mediated polypeptide synthesis in a mitochondrion.